{
  "term_label": "peroxisome proliferator activated receptor signaling pathway",
  "gene_symbol": "FAM120B",
  "gene_name": "Constitutive coactivator of peroxisome proliferator-activated receptor gamma",
  "gene": "UniProtKB:Q96EK7",
  "term_id": "GO:0035357"
}